{
  "term_id": "GO:0002250",
  "term_label": "adaptive immune response",
  "gene_name": "T cell receptor alpha variable 8-2",
  "gene": "UniProtKB:A0A0B4J237",
  "gene_symbol": "TRAV8-2"
}